{
  "term_label": "nucleus",
  "term_id": "GO:0005634",
  "gene": "UniProtKB:Q8WYA1",
  "gene_name": "Basic helix-loop-helix ARNT-like protein 2",
  "gene_symbol": "BMAL2"
}